{
  "gene": "UniProtKB:Q495X7",
  "gene_symbol": "TRIM60",
  "term_label": "cytoplasm",
  "term_id": "GO:0005737",
  "gene_name": "Tripartite motif-containing protein 60"
}